{
  "gene": "UniProtKB:E5RJ46",
  "term_id": "UNKNOWN:0001",
  "term_label": "Unknown molecular function",
  "gene_symbol": "LINC02906",
  "gene_name": "Putative uncharacterized protein LINC02906"
}